{
  "term_id": "GO:0051015",
  "term_label": "actin filament binding",
  "gene_name": "Coronin-6",
  "gene_symbol": "CORO6",
  "gene": "UniProtKB:Q6QEF8"
}